{
  "term_label": "plasma membrane",
  "gene_name": "Leucine-rich repeats and immunoglobulin-like domains protein 3",
  "gene": "UniProtKB:Q6UXM1",
  "term_id": "GO:0005886",
  "gene_symbol": "LRIG3"
}